{
  "term_label": "histone deacetylase binding",
  "gene_name": "Melanoma-associated antigen 8",
  "gene": "UniProtKB:P43361",
  "term_id": "GO:0042826",
  "gene_symbol": "MAGEA8"
}